{
  "gene_symbol": "NDUFC2",
  "term_label": "respiratory chain complex I",
  "gene": "UniProtKB:O95298",
  "gene_name": "NADH dehydrogenase [ubiquinone] 1 subunit C2",
  "term_id": "GO:0045271"
}